{
  "gene": "UniProtKB:Q96F15",
  "gene_name": "GTPase IMAP family member 5",
  "term_label": "Unknown biological process",
  "term_id": "UNKNOWN:0002",
  "gene_symbol": "GIMAP5"
}